{
  "term_label": "RNA polymerase II cis-regulatory region sequence-specific DNA binding",
  "gene_name": "Homeobox expressed in ES cells 1",
  "gene_symbol": "HESX1",
  "gene": "UniProtKB:Q9UBX0",
  "term_id": "GO:0000978"
}